{
  "term_label": "L-glutamate transmembrane transporter activity",
  "gene_symbol": "SLC25A13",
  "term_id": "GO:0005313",
  "gene": "UniProtKB:Q9UJS0",
  "gene_name": "Electrogenic aspartate_glutamate antiporter SLC25A13, mitochondrial"
}